{
  "gene": "UniProtKB:P18206",
  "term_label": "plasma membrane",
  "term_id": "GO:0005886",
  "gene_name": "Vinculin",
  "gene_symbol": "VCL"
}